regulation of type IIa hypersensitivity [GO:0001796] (biological process) Subtypes: negative regulation of type IIa hypersensitivity [GO:0001797], positive regulation of type IIa hypersensitivity [GO:0001798], GO:0001813 Sources: GOC:add, ISBN:0781735149 Definition: Any process that modulates the frequency, rate, or extent of type IIa hypersensitivity, a type of inflammatory response. Relationships: is_a regulation of type II hypersensitivity [GO:0002892]; regulates type IIa hypersensitivity [GO:0001794]